nucleobase-containing small molecule biosynthetic process [GO:0034404] (biological process) Relationships: is a type of nucleobase-containing compound biosynthetic process [GO:0034654]; is a type of small molecule biosynthetic process [GO:0044283]; is a type of nucleobase-containing small molecule metabolic process [GO:0055086] Also known as: nucleobase, nucleoside and nucleotide anabolism, nucleobase, nucleoside and nucleotide biosynthesis, nucleobase, nucleoside and nucleotide formation, nucleobase, nucleoside and nucleotide synthesis Sources: GOC:mah Subtypes: nucleoside biosynthetic process [GO:0009163] Definition: The chemical reactions and pathways resulting in the formation of a nucleobase-containing small molecule: a nucleobase, a nucleoside, or a nucleotide.